{
  "term_id": "GO:0098554",
  "term_label": "cytoplasmic side of endoplasmic reticulum membrane",
  "gene": "UniProtKB:Q8TCT7",
  "gene_symbol": "SPPL2B",
  "gene_name": "Signal peptide peptidase-like 2B"
}